{
  "term_label": "barbed-end actin filament capping",
  "gene": "UniProtKB:P47755",
  "term_id": "GO:0051016",
  "gene_symbol": "CAPZA2",
  "gene_name": "F-actin-capping protein subunit alpha-2"
}